{
  "term_label": "transcription corepressor activity",
  "term_id": "GO:0003714",
  "gene_name": "EP300-interacting inhibitor of differentiation 1",
  "gene_symbol": "EID1",
  "gene": "UniProtKB:Q9Y6B2"
}